{
  "gene": "UniProtKB:P18507",
  "gene_name": "Gamma-aminobutyric acid receptor subunit gamma-2",
  "gene_symbol": "GABRG2",
  "term_id": "GO:0007214",
  "term_label": "gamma-aminobutyric acid signaling pathway"
}